{
  "gene_name": "Single Ig IL-1-related receptor",
  "term_id": "GO:0007166",
  "gene_symbol": "SIGIRR",
  "gene": "UniProtKB:Q6IA17",
  "term_label": "cell surface receptor signaling pathway"
}